{
  "gene_symbol": "MEGF8",
  "term_label": "Unknown cellular component",
  "term_id": "UNKNOWN:0003",
  "gene": "UniProtKB:Q7Z7M0",
  "gene_name": "Multiple epidermal growth factor-like domains protein 8"
}